{
  "gene_name": "H(+)_Cl(-) exchange transporter 3",
  "term_id": "GO:0005769",
  "term_label": "early endosome",
  "gene": "UniProtKB:P51790",
  "gene_symbol": "CLCN3"
}